symbiont-mediated perturbation of host membrane [GO:0141171] (biological process) Also known as: symbiont-mediated disruption of host membrane Subtypes: symbiont-mediated pore formation in host plasma membrane [GO:0044658], symbiont genome entry into host cell via pore formation in plasma membrane [GO:0044694], GO:0052025, symbiont entry into host cell via permeabilization of host membrane [GO:0140267], reorganization of cellular membranes to establish viral sites of replication [GO:0140754], reorganization of host cellular membranes to establish sites of replication [GO:0140755] Relationships: is a type of GO:0052008 References: PMID:14688136, PMID:17043230, PMID:28855258 Definition: The process in which a symbiont effects a change that impairs the structure or function of a host membrane. The host is defined as the larger of the organisms involved in a symbiotic interaction.